{
  "term_id": "GO:0005886",
  "gene": "UniProtKB:Q9Y5I4",
  "term_label": "plasma membrane",
  "gene_symbol": "PCDHAC2",
  "gene_name": "Protocadherin alpha-C2"
}